{
  "term_id": "GO:0000070",
  "gene": "UniProtKB:Q9NRH3",
  "gene_symbol": "TUBG2",
  "term_label": "mitotic sister chromatid segregation",
  "gene_name": "Tubulin gamma-2 chain"
}